{
  "gene_name": "Probable ubiquitin carboxyl-terminal hydrolase FAF-Y",
  "term_id": "GO:0004843",
  "gene_symbol": "USP9Y",
  "gene": "UniProtKB:O00507",
  "term_label": "cysteine-type deubiquitinase activity"
}